{
  "gene": "UniProtKB:A6NE01",
  "gene_symbol": "FAM186A",
  "term_id": "UNKNOWN:0003",
  "term_label": "Unknown cellular component",
  "gene_name": "Protein FAM186A"
}